calcium, potassium:sodium antiporter activity [GO:0008273] (molecular function) Sources: TC:2.A.19.4.1 Relationships: is a type of calcium:sodium antiporter activity [GO:0005432]; is a type of solute:potassium antiporter activity [GO:0022821] Also known as: potassium-dependent sodium/calcium exchanger Definition: Enables the transfer of a solute or solutes from one side of a membrane to the other according to the reaction: Ca2+(in) + K+(in) + Na+(out) = Ca2+(out) + K+(out) + Na+(in).